{
  "gene_name": "ETS-related transcription factor Elf-2",
  "gene": "UniProtKB:Q15723",
  "term_id": "GO:0006357",
  "gene_symbol": "ELF2",
  "term_label": "regulation of transcription by RNA polymerase II"
}